prostate epithelial cord elongation [GO:0060523] (biological process) Relationships: is a type of branch elongation of an epithelium [GO:0060602]; is a type of prostate gland morphogenetic growth [GO:0060737]; is a type of prostate gland epithelium morphogenesis [GO:0060740]; is part of branching involved in prostate gland morphogenesis [GO:0060442] Definition: The developmental growth process in which solid chords of prostate epithelium increase in length. References: PMID:18977204 Sources: GOC:dph